stromule [GO:0010319] (cellular component) References: PMID:15272881, PMID:15699062, PMID:16582010 Relationships: is a type of GO:0110165; is part of plastid envelope [GO:0009526] Definition: Thin filamentous structure extending from the surface of all plastid types examined so far, including chloroplast, proplastid, etioplast, leucoplast, amyloplast, and chromoplast. In general, stromules are more abundant in tissues containing non-green plastids, and in cells containing smaller plastids. The primary function of stromules is still unresolved, although the presence of stromules markedly increases the plastid surface area, potentially increasing transport to and from the cytosol. Other functions of stromules, such as transfer of macromolecules between plastids and starch granule formation in cereal endosperm, may be restricted to particular tissues and cell types. Also known as: Stroma-filled tubule